{
  "gene_name": "Pyrroline-5-carboxylate reductase 1, mitochondrial",
  "gene": "UniProtKB:P32322",
  "term_id": "UNKNOWN:0003",
  "term_label": "Unknown cellular component",
  "gene_symbol": "PYCR1"
}